{
  "gene_symbol": "ZBTB34",
  "gene": "UniProtKB:Q8NCN2",
  "gene_name": "Zinc finger and BTB domain-containing protein 34",
  "term_id": "GO:0005654",
  "term_label": "nucleoplasm"
}